{
  "gene": "UniProtKB:Q92930",
  "term_id": "GO:0005768",
  "gene_name": "Ras-related protein Rab-8B",
  "term_label": "endosome",
  "gene_symbol": "RAB8B"
}